N-acylsphingosine galactosyltransferase activity [GO:0003851] (molecular function) Definition: Catalysis of the reaction: N-acylsphing-4-enine + UDP-alpha-D-galactose = a beta-D-galactosyl-(1<->1')-N-acylsphing-4-enine + H+ + UDP. Sources: EC:2.4.1.47 Also known as: 2-hydroxyacylsphingosine 1-beta-galactosyltransferase activity Relationships: is a type of UDP-galactosyltransferase activity [GO:0035250]